{
  "gene_name": "T-box transcription factor TBX18",
  "term_label": "RNA polymerase II cis-regulatory region sequence-specific DNA binding",
  "gene_symbol": "TBX18",
  "gene": "UniProtKB:O95935",
  "term_id": "GO:0000978"
}